{
  "term_id": "GO:0061844",
  "gene_symbol": "REG3A",
  "term_label": "antimicrobial humoral immune response mediated by antimicrobial peptide",
  "gene_name": "Regenerating islet-derived protein 3-alpha",
  "gene": "UniProtKB:Q06141"
}